radial spoke neck [GO:0120343] (cellular component) References: PMID:22754630 Sources: GOC:krc Definition: The radial spoke neck is a complex that connects the spoke stalk to the head. Relationships: is a type of protein-containing complex [GO:0032991]; is part of radial spoke [GO:0001534]